{
  "gene": "UniProtKB:Q86WN2",
  "term_id": "GO:0060337",
  "gene_name": "Interferon epsilon",
  "term_label": "type I interferon-mediated signaling pathway",
  "gene_symbol": "IFNE"
}